{
  "term_id": "GO:0016020",
  "term_label": "membrane",
  "gene_name": "Chemokine-like factor",
  "gene": "UniProtKB:Q9UBR5",
  "gene_symbol": "CKLF"
}